{
  "gene_name": "Protein unc-119 homolog A",
  "term_label": "lipid binding",
  "gene_symbol": "UNC119",
  "gene": "UniProtKB:Q13432",
  "term_id": "GO:0008289"
}